{
  "term_label": "cytoplasm",
  "term_id": "GO:0005737",
  "gene_symbol": "SKOR2",
  "gene_name": "SKI family transcriptional corepressor 2",
  "gene": "UniProtKB:Q2VWA4"
}